{
  "gene_name": "Phosphoinositide 3-kinase regulatory subunit 4",
  "gene": "UniProtKB:Q99570",
  "term_id": "GO:0071561",
  "gene_symbol": "PIK3R4",
  "term_label": "nucleus-vacuole junction"
}